glycine N-methyltransferase activity [GO:0017174] (MF) Definition: Catalysis of the reaction: S-adenosyl-L-methionine + glycine = S-adenosyl-L-homocysteine + sarcosine. Sources: EC:2.1.1.20 Also known as: GNMT, S-adenosyl-L-methionine:glycine N-methyltransferase activity, S-adenosyl-L-methionine:glycine methyltransferase activity, glycine methyltransferase activity Relationships: is a type of N-methyltransferase activity [GO:0008170]; is a type of S-adenosylmethionine-dependent methyltransferase activity [GO:0008757]